{
  "gene_symbol": "S100A12",
  "gene_name": "Protein S100-A12",
  "gene": "UniProtKB:P80511",
  "term_label": "calcium-dependent protein binding",
  "term_id": "GO:0048306"
}